{
  "gene_name": "Delta-1-pyrroline-5-carboxylate synthase",
  "gene": "UniProtKB:P54886",
  "gene_symbol": "ALDH18A1",
  "term_id": "GO:0004350",
  "term_label": "glutamate-5-semialdehyde dehydrogenase activity"
}